{
  "term_id": "UNKNOWN:0003",
  "gene_symbol": "LOC344065",
  "term_label": "Unknown cellular component",
  "gene_name": "KRAB domain-containing protein (Fragment)",
  "gene": "UniProtKB:A0A087WZK3"
}